{
  "term_id": "GO:0019532",
  "term_label": "oxalate transport",
  "gene": "UniProtKB:P58743",
  "gene_symbol": "SLC26A5",
  "gene_name": "Prestin"
}